{
  "term_label": "Unknown cellular component",
  "gene_name": "Protein-lysine methyltransferase METTL21C",
  "gene_symbol": "METTL21C",
  "gene": "UniProtKB:Q5VZV1",
  "term_id": "UNKNOWN:0003"
}